{
  "gene_symbol": "CD300C",
  "gene_name": "CMRF35-like molecule 6",
  "gene": "UniProtKB:Q08708",
  "term_id": "GO:0007165",
  "term_label": "signal transduction"
}